{
  "gene": "UniProtKB:P51686",
  "term_label": "C-C chemokine receptor activity",
  "term_id": "GO:0016493",
  "gene_symbol": "CCR9",
  "gene_name": "C-C chemokine receptor type 9"
}